{
  "gene": "UniProtKB:Q9H0M4",
  "term_label": "Unknown molecular function",
  "gene_symbol": "ZCWPW1",
  "gene_name": "Zinc finger CW-type PWWP domain protein 1",
  "term_id": "UNKNOWN:0001"
}